tricarboxylic acid biosynthetic process [GO:0072351] (biological process) Also known as: tricarboxylate biosynthesis, tricarboxylate biosynthetic process, tricarboxylic acid anabolism, tricarboxylic acid biosynthesis, tricarboxylic acid formation, tricarboxylic acid synthesis Subtypes: pyrroloquinoline quinone biosynthetic process [GO:0018189], aerobactin biosynthetic process [GO:0019270], nicotianamine biosynthetic process [GO:0030418], GO:1900868, GO:1901855, coenzyme gamma-F420-2 biosynthetic process [GO:2001121] Sources: GOC:mah Definition: The chemical reactions and pathways resulting in the formation of dicarboxylic acids, any organic acid containing three carboxyl (-COOH) groups. Relationships: is a type of carboxylic acid biosynthetic process [GO:0046394]; is a type of tricarboxylic acid metabolic process [GO:0072350]